{
  "term_label": "regulation of transcription by RNA polymerase II",
  "gene": "UniProtKB:Q5JVG2",
  "gene_symbol": "ZNF484",
  "term_id": "GO:0006357",
  "gene_name": "Zinc finger protein 484"
}